phosphoglycolate phosphatase activity [GO:0008967] (molecular function) Definition: Catalysis of the reaction: 2-phosphoglycolate + H2O = glycolate + phosphate. Sources: EC:3.1.3.18, RHEA:14369 Also known as: 2-phosphoglycolate phosphatase activity, 2-phosphoglycolate phosphohydrolase activity, P-glycolate phosphatase activity, phosphoglycolate hydrolase activity, phosphoglycollate phosphatase activity Relationships: is a type of phosphatase activity [GO:0016791]